{
  "term_label": "extracellular space",
  "gene_name": "Prostate-associated microseminoprotein",
  "gene_symbol": "MSMP",
  "term_id": "GO:0005615",
  "gene": "UniProtKB:Q1L6U9"
}